venom-mediated perturbation of voltage-gated sodium channel activity [GO:0044492] (biological process) Also known as: envenomation resulting in modulation of voltage-gated sodium channel activity in another organism, envenomation resulting in modulation of voltage-gated sodium channel activity in other organism References: PMID:21781281 Sources: GOC:fj, GOC:jl Subtypes: venom-mediated inhibition of voltage-gated sodium channel activity [GO:0044493], venom-mediated activation of voltage-gated sodium channel activity [GO:0044494] Definition: A process in which an organism alters or subverts the activity of a voltage-gated sodium channel in another organism via the action of a venom. Relationships: is a type of venom-mediated perturbation of ion channel activity [GO:0044560]